{
  "gene_symbol": "EVL",
  "gene_name": "Ena_VASP-like protein",
  "gene": "UniProtKB:Q9UI08",
  "term_id": "GO:0008154",
  "term_label": "actin polymerization or depolymerization"
}